{
  "term_label": "p38MAPK cascade",
  "gene_symbol": "MAP3K6",
  "term_id": "GO:0038066",
  "gene_name": "Mitogen-activated protein kinase kinase kinase 6",
  "gene": "UniProtKB:O95382"
}